{
  "gene": "UniProtKB:Q9NS26",
  "term_label": "Unknown molecular function",
  "gene_name": "Sperm protein associated with the nucleus on the X chromosome A",
  "term_id": "UNKNOWN:0001",
  "gene_symbol": "SPANXA2"
}